{
  "term_id": "GO:0004980",
  "gene_symbol": "MC3R",
  "gene": "UniProtKB:P41968",
  "term_label": "melanocyte-stimulating hormone receptor activity",
  "gene_name": "Melanocortin receptor 3"
}